{
  "gene_name": "V-set and transmembrane domain-containing protein 2B",
  "term_id": "UNKNOWN:0002",
  "term_label": "Unknown biological process",
  "gene": "UniProtKB:A6NLU5",
  "gene_symbol": "VSTM2B"
}